L-phenylalanine biosynthetic process from chorismate via L-arogenate [GO:0033586] (biological process) Also known as: L-phenylalanine anabolism from chorismate via L-arogenate, L-phenylalanine biosynthesis from chorismate via L-arogenate, L-phenylalanine formation from chorismate via L-arogenate, L-phenylalanine synthesis from chorismate via L-arogenate Relationships: is a type of L-phenylalanine biosynthetic process [GO:0009094]; is a type of chorismate metabolic process [GO:0046417] Definition: The chemical reactions and pathways resulting in the formation of L-phenylalanine from other compounds, including chorismate, via the intermediate L-arogenate. Sources: GOC:go_curators